{
  "gene_name": "FAS-associated factor 1",
  "term_id": "GO:0043130",
  "gene_symbol": "FAF1",
  "gene": "UniProtKB:Q9UNN5",
  "term_label": "ubiquitin binding"
}